L-cystine transport [GO:0015811] (biological process) Sources: GOC:go_curators, ISBN:0198506732 Definition: The directed movement of L-cystine (also known as dicysteine) into, out of or within a cell, or between cells, by means of some agent such as a transporter or pore. Subtypes: L-cystine transmembrane transport from lysosomal lumen to cytosol [GO:1904919] Relationships: is a type of sulfur amino acid transport [GO:0000101]; is a type of neutral amino acid transport [GO:0015804]; is a type of GO:0015807; is_a GO:0072337